{
  "gene": "UniProtKB:Q96N67",
  "term_id": "UNKNOWN:0003",
  "term_label": "Unknown cellular component",
  "gene_symbol": "DOCK7",
  "gene_name": "Dedicator of cytokinesis protein 7"
}